{
  "gene_name": "Mothers against decapentaplegic homolog 5",
  "term_label": "heteromeric SMAD protein complex",
  "gene": "UniProtKB:Q99717",
  "gene_symbol": "SMAD5",
  "term_id": "GO:0071144"
}